lung lobe morphogenesis [GO:0060463] (BP) Definition: The process in which the anatomical structures of a lung lobe are generated and organized. A lung lobe is a projection that extends from the lung. Relationships: is a type of anatomical structure morphogenesis [GO:0009653]; is part of lung morphogenesis [GO:0060425]; is part of lung lobe development [GO:0060462] Sources: GOC:dph